telomere localization [GO:0034397] (biological process) Sources: GOC:mah, GOC:vw Relationships: is a type of chromosome localization [GO:0050000] Subtypes: GO:0034398, GO:0045141, mitotic telomere clustering and tethering at nuclear periphery [GO:0120109], interphase mitotic telomere clustering [GO:0120110] Also known as: telomere localisation Definition: Any process in which a telomere is transported to, and/or maintained in, a specific location.